{
  "gene": "UniProtKB:P0DMN0",
  "gene_name": "Sulfotransferase 1A4",
  "term_label": "sulfation",
  "term_id": "GO:0051923",
  "gene_symbol": "SULT1A4"
}